regulation of type B pancreatic cell development [GO:2000074] (biological process) Relationships: is a type of GO:0060284; regulates GO:0003323 Subtypes: negative regulation of type B pancreatic cell development [GO:2000077], GO:2000078 Also known as: regulation of pancreatic B cell development, regulation of pancreatic beta cell development Sources: GOC:obol, GOC:yaf Definition: Any process that modulates the frequency, rate or extent of pancreatic B cell development.